rolling circle viral DNA replication [GO:0039682] (biological process) Definition: A process of unidirectional viral DNA replication that takes place on a circular DNA to rapidly produce numerous copies of the viral genome. Involves creating a nick in one strand of the circular DNA molecule at the origin of replication. DNA is then synthesized by DNA polymerase. Using the non-nicked strand as a template, replication proceeds around the circular DNA molecule, displacing the nicked strand as single-stranded DNA. Sources: GOC:bf, GOC:jl, VZ:915, Wikipedia:Rolling_circle_replication Relationships: is a type of viral DNA strand displacement replication [GO:0039687] Subtypes: rolling circle double-stranded viral DNA replication [GO:0039683], rolling circle single-stranded viral DNA replication [GO:0039684]